estradiol 17-alpha-dehydrogenase [NAD(P)+] activity [GO:0047881] (molecular function) Definition: Catalysis of the reaction: estradiol-17-alpha + NAD(P)+ = estrone + NAD(P)H + H+. Relationships: is a type of steroid dehydrogenase activity, acting on the CH-OH group of donors, NAD or NADP as acceptor [GO:0033764] Also known as: estradiol 17a-dehydrogenase activity, 17alpha-estradiol dehydrogenase activity, 17alpha-hydroxy steroid dehydrogenase activity, 17alpha-hydroxy steroid oxidoreductase activity, 17alpha-hydroxysteroid oxidoreductase activity, 17alpha-hydroxysteroid:NAD(P)+ 17-oxidoreductase activity, estradiol 17alpha-dehydrogenase activity, estradiol 17alpha-oxidoreductase activity Sources: EC:1.1.1.148